{
  "gene_symbol": "ATP5MC1",
  "gene_name": "ATP synthase F(0) complex subunit C1, mitochondrial",
  "gene": "UniProtKB:P05496",
  "term_label": "proton-transporting ATP synthase complex",
  "term_id": "GO:0045259"
}